substance P secretion [GO:1990772] (biological process) Regulation: regulated by GO:1904458; negatively regulated by GO:1904459; positively regulated by positive regulation of substance P secretion [GO:1904460] Subtypes: substance P secretion, neurotransmission [GO:1990793] Definition: The regulated release of substance P, a peptide hormone that is involved in neurotransmission, inflammation, and antimicrobial activity. Relationships: is a type of GO:0030072 References: PMID:11278900